{
  "term_label": "Unknown molecular function",
  "term_id": "UNKNOWN:0001",
  "gene_name": "Intermembrane lipid transfer protein VPS13A",
  "gene": "UniProtKB:Q96RL7",
  "gene_symbol": "VPS13A"
}